porous cell septum [GO:0000934] (cellular component) Relationships: is a type of cell septum [GO:0030428] Subtypes: dolipore septum [GO:0000937] Sources: GOC:clt Also known as: porous septum Definition: A septum or cross wall which does not entirely span the space between two portions of cell wall and may contain a specialized central pore structure. A porous septum allows the movement of organelles and/or cytoplasm between compartments.